{
  "gene": "UniProtKB:P32929",
  "gene_symbol": "CTH",
  "term_label": "pyridoxal phosphate binding",
  "term_id": "GO:0030170",
  "gene_name": "Cystathionine gamma-lyase"
}